{
  "gene_symbol": "CCN2",
  "gene_name": "CCN family member 2",
  "term_id": "GO:0007165",
  "gene": "UniProtKB:P29279",
  "term_label": "signal transduction"
}